{
  "gene_symbol": "RTP2",
  "term_label": "olfactory receptor binding",
  "gene": "UniProtKB:Q5QGT7",
  "term_id": "GO:0031849",
  "gene_name": "Receptor-transporting protein 2"
}